myeloid cell differentiation [GO:0030099] (biological process) Subtypes: myeloid leukocyte differentiation [GO:0002573], thrombocyte differentiation [GO:0002574], erythrocyte differentiation [GO:0030218], megakaryocyte differentiation [GO:0030219], GO:0030220 Definition: The process in which a relatively unspecialized myeloid precursor cell acquires the specialized features of any cell of the myeloid leukocyte, megakaryocyte, thrombocyte, or erythrocyte lineages. Regulation: RO_0002211 by regulation of myeloid cell differentiation [GO:0045637]; negatively regulated by negative regulation of myeloid cell differentiation [GO:0045638]; positively regulated by positive regulation of myeloid cell differentiation [GO:0045639] Sources: GOC:add, ISBN:0781735149 Relationships: is a type of cell differentiation [GO:0030154]; is part of hemopoiesis [GO:0030097]